{
  "gene": "UniProtKB:Q9NQR4",
  "term_label": "Unknown cellular component",
  "gene_symbol": "NIT2",
  "term_id": "UNKNOWN:0003",
  "gene_name": "Omega-amidase NIT2"
}